positive regulation of hydrolase activity [GO:0051345] (biological process) Definition: Any process that activates or increases the frequency, rate or extent of hydrolase activity, the catalysis of the hydrolysis of various bonds. Also known as: hydrolase activator, up regulation of hydrolase activity, up-regulation of hydrolase activity, upregulation of hydrolase activity, activation of hydrolase activity, stimulation of hydrolase activity Sources: GOC:ai Relationships: is a type of positive regulation of catalytic activity [GO:0043085]; is a type of GO:0051336; RO_0002213 hydrolase activity [GO:0016787] Subtypes: positive regulation of phosphatase activity [GO:0010922], positive regulation of peptidase activity [GO:0010952], positive regulation of GTPase activity [GO:0043547], positive regulation of lipase activity [GO:0060193], positive regulation of phosphodiesterase I activity [GO:1902800], GO:1903017, positive regulation of lysozyme activity [GO:1903592], positive regulation of beta-galactosidase activity [GO:1903771]